death-inducing signaling complex assembly [GO:0071550] (biological process) Definition: A process of protein complex assembly in which the arrangement and bonding together of the set of components that form the protein complex is mediated by a death domain (DD) interaction, as part of the extrinsic apoptotic signaling pathway. Sources: GOC:amm, GOC:mtg_apoptosis, InterPro:IPR000488 Also known as: DD-mediated complex assembly, DISC assembly, DISC formation, death domain-mediated complex assembly, death domain-mediated complex assembly involved in extrinsic apoptotic pathway, death-inducing signaling complex formation, death-inducing signalling complex assembly Relationships: is a type of GO:0065003; is part of extrinsic apoptotic signaling pathway [GO:0097191] Subtypes: TRAIL death-inducing signaling complex assembly [GO:1903074] Regulation: regulated by regulation of death-inducing signaling complex assembly [GO:1903072]; negatively regulated by negative regulation of death-inducing signaling complex assembly [GO:1903073]